{
  "gene_name": "Guanine nucleotide-binding protein G(i) subunit alpha-2",
  "gene_symbol": "GNAI2",
  "gene": "UniProtKB:P04899",
  "term_label": "G protein-coupled adenosine receptor signaling pathway",
  "term_id": "GO:0001973"
}